UDP-N-acetylmuramoyl-L-alanyl-D-glutamate--D-lysine ligase activity [GO:0102195] (molecular function) Relationships: is a type of acid-amino acid ligase activity [GO:0016881] Definition: Catalysis of the reaction: UDP-N-acetylmuramoyl-L-alanyl-D-glutamate + D-lysinium(1+) + ATP = UDP-N-acetylmuramoyl-L-alanyl-gamma-D-glutamyl-D-lysine + ADP + hydrogenphosphate + H+. Sources: EC:6.3.2.37, GOC:pz